{
  "term_label": "cytoplasm",
  "gene": "UniProtKB:O14787",
  "term_id": "GO:0005737",
  "gene_name": "Transportin-2",
  "gene_symbol": "TNPO2"
}